regulation of (R)-carnitine transmembrane transport [GO:1902272] (biological process) Relationships: is a type of regulation of transmembrane transport [GO:0034762]; regulates GO:1902270 Subtypes: GO:1902273, positive regulation of (R)-carnitine transmembrane transport [GO:1902274] References: PMID:23755272 Sources: GOC:TermGenie Definition: Any process that modulates the frequency, rate or extent of (R)-carnitine transmembrane transport.